{
  "gene": "UniProtKB:O43248",
  "term_label": "nucleus",
  "gene_symbol": "HOXC11",
  "term_id": "GO:0005634",
  "gene_name": "Homeobox protein Hox-C11"
}